{
  "gene_name": "DnaJ homolog subfamily C member 18",
  "term_label": "cellular response to misfolded protein",
  "term_id": "GO:0071218",
  "gene": "UniProtKB:Q9H819",
  "gene_symbol": "DNAJC18"
}